{
  "gene_symbol": "ATP23",
  "term_label": "mitochondrial proton-transporting ATP synthase complex assembly",
  "gene": "UniProtKB:Q9Y6H3",
  "gene_name": "Mitochondrial inner membrane protease ATP23 homolog",
  "term_id": "GO:0033615"
}